{
  "gene_name": "Neurogenin-2",
  "gene": "UniProtKB:Q9H2A3",
  "gene_symbol": "NEUROG2",
  "term_id": "GO:0061564",
  "term_label": "axon development"
}